AMP salvage [GO:0044209] (biological process) Also known as: AMP biosynthetic process via salvage pathway, adenosine monophosphate salvage References: PMID:8917457, PMID:9864350 Sources: GOC:ecd, GOC:jl Definition: The chemical reactions and pathways resulting in the formation of adenosine monophosphate (AMP) from derivatives of it (either adenine, ADP or adenosine 3',5'-bisphosphate) without de novo synthesis. Relationships: is a type of AMP biosynthetic process [GO:0006167]; is a type of purine ribonucleotide salvage [GO:0106380]